thiopurine S-methyltransferase activity [GO:0008119] (molecular function) Definition: Catalysis of the reaction: S-adenosyl-L-methionine + a thiopurine = S-adenosyl-L-homocysteine + a thiopurine S-methylether. Sources: EC:2.1.1.67 Also known as: 6-thiopurine transmethylase activity, S-adenosyl-L-methionine:thiopurine S-methyltransferase activity, TPMT, mercaptopurine methyltransferase activity, thiopurine methyltransferase activity Relationships: is a type of GO:0008172; is a type of S-adenosylmethionine-dependent methyltransferase activity [GO:0008757]